{
  "gene": "UniProtKB:Q86WI3",
  "gene_symbol": "NLRC5",
  "term_id": "GO:0005634",
  "gene_name": "Protein NLRC5",
  "term_label": "nucleus"
}